{
  "gene_symbol": "DEFB135",
  "term_id": "UNKNOWN:0003",
  "term_label": "Unknown cellular component",
  "gene": "UniProtKB:Q30KP9",
  "gene_name": "Beta-defensin 135"
}